{
  "term_id": "UNKNOWN:0003",
  "gene": "UniProtKB:Q6N043",
  "gene_symbol": "ZNF280D",
  "gene_name": "Zinc finger protein 280D",
  "term_label": "Unknown cellular component"
}